{
  "gene": "UniProtKB:O60306",
  "gene_symbol": "AQR",
  "gene_name": "RNA helicase aquarius",
  "term_id": "UNKNOWN:0002",
  "term_label": "Unknown biological process"
}